{
  "gene_symbol": "THYN1",
  "gene": "UniProtKB:Q9P016",
  "term_label": "Unknown molecular function",
  "term_id": "UNKNOWN:0001",
  "gene_name": "Thymocyte nuclear protein 1"
}